{
  "gene_symbol": "SLC38A4",
  "term_id": "GO:0005886",
  "term_label": "plasma membrane",
  "gene": "UniProtKB:Q969I6",
  "gene_name": "Sodium-coupled neutral amino acid transporter 4"
}